anaerobic L-alanine catabolic process [GO:0019667] (biological process) Also known as: L-alanine fermentation Definition: The anaerobic chemical reactions and pathways resulting in the breakdown of L-alanine, yielding energy in the form of ATP. Sources: GOC:jl Relationships: is a type of anaerobic amino acid catabolic process [GO:0019665]; is a type of GO:0042853; is part of anaerobic catabolism of pairs of amino acids [GO:0019668]